centrolateral pattern formation [GO:0097353] (BP) Relationships: is_a regionalization [GO:0003002] Also known as: mediolateral pattern formation Sources: GOC:dsz Definition: The regionalization process in which the areas along the centrolateral axis are established that will lead to differences in cell differentiation, or in which cells interpret a specific environment.